{
  "term_id": "GO:0034982",
  "gene_name": "Mitochondrial inner membrane protease ATP23 homolog",
  "gene": "UniProtKB:Q9Y6H3",
  "term_label": "mitochondrial protein processing",
  "gene_symbol": "ATP23"
}